{
  "term_label": "establishment of protein localization",
  "term_id": "GO:0045184",
  "gene_name": "WD repeat-containing and planar cell polarity effector protein fritz homolog",
  "gene": "UniProtKB:O95876",
  "gene_symbol": "WDPCP"
}